{
  "term_label": "Unknown molecular function",
  "term_id": "UNKNOWN:0001",
  "gene_symbol": "BMF",
  "gene": "UniProtKB:Q96LC9",
  "gene_name": "Bcl-2-modifying factor"
}